ATPase-coupled carboxylic acid transmembrane transporter activity [GO:0033284] (MF) Definition: Enables the transfer of a solute or solutes from one side of a membrane to the other according to the reaction: ATP + H2O + carboxylic acid(out/in) = ADP + phosphate + carboxylic acid(in/out). Sources: GOC:mlg Also known as: ATP-dependent carboxylic acid transporter activity, carboxylic acid-transporting ATPase activity Relationships: is a type of ATPase-coupled transmembrane transporter activity [GO:0042626]; is_a carboxylic acid transmembrane transporter activity [GO:0046943] Subtypes: GO:0015436, ATPase-coupled L-glutamine transmembrane transporter activity [GO:0015599], ABC-type cysteine transporter activity [GO:0033230], ABC-type D-methionine transporter activity [GO:0033232], ATPase-coupled monocarboxylic acid transmembrane transporter activity [GO:0033285]